{
  "gene_symbol": "LEAP2",
  "gene_name": "Liver-expressed antimicrobial peptide 2",
  "term_id": "UNKNOWN:0003",
  "gene": "UniProtKB:Q969E1",
  "term_label": "Unknown cellular component"
}